TRAM-dependent toll-like receptor signaling pathway [GO:0035668] (biological process) Subtypes: TRAM-dependent toll-like receptor 4 signaling pathway [GO:0035669] References: PMID:14556004 Sources: GOC:BHF Also known as: TRAM-dependent TLR signaling pathway, TRAM-dependent toll-like receptor signalling pathway Relationships: is a type of MyD88-independent toll-like receptor signaling pathway [GO:0002756] Definition: The series of molecular signals initiated by a ligand binding to a toll-like receptor where the TRAM adaptor mediates transduction of the signal. Toll-like receptors directly bind pattern motifs from a variety of microbial sources to initiate an innate immune response.